{
  "term_id": "GO:0007015",
  "term_label": "actin filament organization",
  "gene_symbol": "TPM4",
  "gene": "UniProtKB:P67936",
  "gene_name": "Tropomyosin alpha-4 chain"
}